{
  "gene_symbol": "GPRASP1",
  "gene": "UniProtKB:Q5JY77",
  "gene_name": "G-protein coupled receptor-associated sorting protein 1",
  "term_id": "GO:0005634",
  "term_label": "nucleus"
}